{
  "term_id": "UNKNOWN:0002",
  "gene_name": "Nuclear envelope integral membrane protein 1",
  "term_label": "Unknown biological process",
  "gene": "UniProtKB:O14524",
  "gene_symbol": "NEMP1"
}